regulation of premature acrosome loss [GO:0061949] (biological process) Definition: Any process that modulates the rate, frequency or extent of the discharge, by sperm, of a single, anterior secretory granule before the sperm reaches to the zona pellucida of the oocyte. The process begins with the fusion of the outer acrosomal membrane with the sperm plasma membrane and ends with the exocytosis of the acrosomal contents. References: PMID:22228629, PMID:23430248 Relationships: is a type of regulation of reproductive process [GO:2000241]; regulates GO:0061948 Subtypes: negative regulation of premature acrosome loss [GO:0061950]